{
  "gene": "UniProtKB:O15068",
  "term_id": "GO:0005085",
  "gene_name": "Guanine nucleotide exchange factor DBS",
  "gene_symbol": "MCF2L",
  "term_label": "guanyl-nucleotide exchange factor activity"
}